{
  "term_id": "GO:0002323",
  "term_label": "natural killer cell activation involved in immune response",
  "gene_name": "Interferon epsilon",
  "gene": "UniProtKB:Q86WN2",
  "gene_symbol": "IFNE"
}